{
  "gene_symbol": "FAM13B",
  "term_label": "Unknown molecular function",
  "gene": "UniProtKB:Q9NYF5",
  "term_id": "UNKNOWN:0001",
  "gene_name": "Protein FAM13B"
}